{
  "term_id": "GO:0004725",
  "gene_symbol": "PTPN14",
  "gene": "UniProtKB:Q15678",
  "gene_name": "Tyrosine-protein phosphatase non-receptor type 14",
  "term_label": "protein tyrosine phosphatase activity"
}